{
  "term_label": "negative regulation of cholesterol storage",
  "gene": "UniProtKB:Q03181",
  "gene_name": "Peroxisome proliferator-activated receptor delta",
  "term_id": "GO:0010887",
  "gene_symbol": "PPARD"
}